{
  "gene_name": "Cysteine-rich protein 2-binding protein",
  "term_label": "Unknown cellular component",
  "gene_symbol": "KAT14",
  "gene": "UniProtKB:Q9H8E8",
  "term_id": "UNKNOWN:0003"
}